rRNA 3'-end processing [GO:0031125] (biological process) Subtypes: endonucleolytic cleavage to generate mature 3'-end of SSU-rRNA from (SSU-rRNA, 5.8S rRNA, LSU-rRNA) [GO:0000461], exonucleolytic trimming to generate mature 3'-end of 5.8S rRNA from tricistronic rRNA transcript (SSU-rRNA, 5.8S rRNA, LSU-rRNA) [GO:0000467], generation of mature 3'-end of LSU-rRNA from tricistronic rRNA transcript (SSU-rRNA, 5.8S rRNA, LSU-rRNA) [GO:0000468], generation of mature 3'-end of 5S rRNA generated by RNA polymerase III [GO:0002107] Also known as: rRNA 3' end processing Sources: GOC:mah Definition: Any process involved in forming the mature 3' end of an rRNA molecule. Relationships: is a type of rRNA processing [GO:0006364]; is a type of RNA 3'-end processing [GO:0031123]